L-2-amino-4-chloropent-4-enoate dehydrochlorinase activity [GO:0047460] (molecular function) Definition: Catalysis of the reaction: L-2-amino-4-chloropent-4-enoate + H2O = 2-oxopent-4-enoate + chloride + H+ + NH4. Sources: EC:4.5.1.4, RHEA:11620 Also known as: L-2-amino-4-chloro-4-pentenoate dehalogenase activity, L-2-amino-4-chloropent-4-enoate chloride-lyase (adding H2O; deaminating; 2-oxopent-4-enoate-forming), L-2-amino-4-chloropent-4-enoate chloride-lyase (deaminating) Relationships: is a type of carbon-halide lyase activity [GO:0016848]